{
  "term_label": "Unknown molecular function",
  "gene_symbol": "CYTIP",
  "term_id": "UNKNOWN:0001",
  "gene_name": "Cytohesin-interacting protein",
  "gene": "UniProtKB:O60759"
}